{
  "gene_name": "TSC22 domain family protein 4",
  "gene": "UniProtKB:Q9Y3Q8",
  "gene_symbol": "TSC22D4",
  "term_label": "response to osmotic stress",
  "term_id": "GO:0006970"
}